{
  "gene": "UniProtKB:Q96QU6",
  "term_id": "UNKNOWN:0003",
  "gene_symbol": "ACCS",
  "gene_name": "1-aminocyclopropane-1-carboxylate synthase-like protein 1",
  "term_label": "Unknown cellular component"
}